myoblast division [GO:0014872] (biological process) Sources: CL:0000056, GOC:ef, GOC:mtg_muscle Relationships: is a type of cell division [GO:0051301] Definition: The process resulting in the physical partitioning and separation of a myoblast into daughter cells. A myoblast is a mononucleate cell type that, by fusion with other myoblasts, gives rise to the myotubes that eventually develop into skeletal muscle fibers.